{
  "term_label": "DNA-binding transcription factor activity",
  "gene_symbol": "ZNF613",
  "gene": "UniProtKB:Q6PF04",
  "gene_name": "Zinc finger protein 613",
  "term_id": "GO:0003700"
}